{
  "gene_name": "NF-kappa-B inhibitor-like protein 1",
  "gene_symbol": "NFKBIL1",
  "term_id": "GO:0005634",
  "term_label": "nucleus",
  "gene": "UniProtKB:Q9UBC1"
}